{
  "gene_symbol": "PRDM16",
  "gene": "UniProtKB:Q9HAZ2",
  "term_id": "GO:0005634",
  "term_label": "nucleus",
  "gene_name": "Histone-lysine N-methyltransferase PRDM16"
}